bacterial-type flagellum-dependent cell motility [GO:0071973] (biological process) Regulation: RO_0002211 by regulation of bacterial-type flagellum-dependent cell motility [GO:1902021]; negatively regulated by negative regulation of bacterial-type flagellum-dependent cell motility [GO:1902201] Relationships: is a type of archaeal or bacterial-type flagellum-dependent cell motility [GO:0097588] Subtypes: bacterial-type flagellum-dependent swimming motility [GO:0071977], bacterial-type flagellum-dependent swarming motility [GO:0071978] Definition: Cell motility due to the motion of one or more bacterial-type flagella. A bacterial-type flagellum is a motor complex composed of an extracellular helical protein filament coupled to a rotary motor embedded in the cell envelope. Also known as: flagellin-based flagellar cell motility, bacterial-type flagellar cell motility Sources: GOC:cilia, GOC:krc, GOC:mah